{
  "gene": "UniProtKB:Q01638",
  "term_id": "GO:0005886",
  "gene_symbol": "IL1RL1",
  "term_label": "plasma membrane",
  "gene_name": "Interleukin-1 receptor-like 1"
}